proline-tRNA ligase activity [GO:0004827] (molecular function) Also known as: prolyl-tRNA synthetase activity, L-proline:tRNAPro ligase (AMP-forming), proline translase activity, prolinyl-tRNA ligase activity, prolyl-s-RNA synthetase activity, prolyl-transfer ribonucleate synthetase activity, prolyl-transfer ribonucleic acid synthetase activity, prolyl-transferRNA synthetase activity Sources: EC:6.1.1.15 Definition: Catalysis of the reaction: ATP + L-proline + tRNA(Pro) = AMP + diphosphate + L-prolyl-tRNA(Pro). Relationships: is a type of aminoacyl-tRNA ligase activity [GO:0004812]